{
  "gene_symbol": "CYP2W1",
  "gene_name": "Cytochrome P450 2W1",
  "gene": "UniProtKB:Q8TAV3",
  "term_id": "GO:0006082",
  "term_label": "organic acid metabolic process"
}